myosin VI heavy chain binding [GO:0070854] (molecular function) Sources: GOC:sart Definition: Binding to a heavy chain of a myosin VI complex. Subtypes: GO:0070855 Relationships: is a type of GO:0032036; is_a myosin VI binding [GO:0070853]